{
  "gene_name": "Nucleolar MIF4G domain-containing protein 1",
  "term_id": "GO:0042274",
  "gene_symbol": "NOM1",
  "gene": "UniProtKB:Q5C9Z4",
  "term_label": "ribosomal small subunit biogenesis"
}